{
  "term_label": "endoplasmic reticulum",
  "term_id": "GO:0005783",
  "gene_symbol": "ALOX5AP",
  "gene": "UniProtKB:P20292",
  "gene_name": "Arachidonate 5-lipoxygenase-activating protein"
}